{
  "gene_symbol": "GRIN1",
  "term_id": "GO:0004972",
  "gene": "UniProtKB:Q05586",
  "gene_name": "Glutamate receptor ionotropic, NMDA 1",
  "term_label": "NMDA glutamate receptor activity"
}